{
  "gene_name": "Phospholipase ABHD3",
  "gene": "UniProtKB:Q8WU67",
  "gene_symbol": "ABHD3",
  "term_label": "phosphatidylcholine metabolic process",
  "term_id": "GO:0046470"
}